{
  "gene": "UniProtKB:P47710",
  "gene_name": "Alpha-S1-casein",
  "term_label": "Unknown molecular function",
  "gene_symbol": "CSN1S1",
  "term_id": "UNKNOWN:0001"
}